{
  "term_id": "GO:0031298",
  "gene_name": "Calmodulin-regulated spectrin-associated protein 3",
  "term_label": "replication fork protection complex",
  "gene_symbol": "CAMSAP3",
  "gene": "UniProtKB:Q9P1Y5"
}